response to trichodermin [GO:1901324] (biological process) Relationships: is a type of response to ether [GO:0045472] Definition: Any process that results in a change in state or activity of a cell or an organism (in terms of movement, secretion, enzyme production, gene expression, etc.) as a result of a trichodermin stimulus. Sources: GOC:TermGenie Subtypes: cellular response to trichodermin [GO:0072744]